{
  "gene_name": "TBCC domain-containing protein 1",
  "term_label": "Unknown molecular function",
  "term_id": "UNKNOWN:0001",
  "gene_symbol": "TBCCD1",
  "gene": "UniProtKB:Q9NVR7"
}